{
  "gene_symbol": "SFXN1",
  "gene": "UniProtKB:Q9H9B4",
  "term_label": "mitochondrial inner membrane",
  "gene_name": "Sideroflexin-1",
  "term_id": "GO:0005743"
}